cardiac muscle cell action potential involved in contraction [GO:0086002] (biological process) Definition: An action potential that occurs in a cardiac muscle cell and is involved in its contraction. Subtypes: ventricular cardiac muscle cell action potential [GO:0086005], atrial cardiac muscle cell action potential [GO:0086014] Sources: GOC:BHF, GOC:mtg_cardiac_conduct_nov11 Relationships: is a type of cardiac muscle cell action potential [GO:0086001]; is part of cardiac muscle cell contraction [GO:0086003]